negative regulation of ERK5 cascade [GO:0070377] (biological process) Sources: GOC:add, ISBN:0121245462, ISBN:0896039986 Definition: Any process that stops, prevents, or reduces the frequency, rate or extent of signal transduction mediated by the ERK5 cascade. Also known as: down regulation of BMK cascade, down-regulation of BMK cascade, downregulation of BMK cascade, negative regulation of BMK cascade, negative regulation of BMK signaling pathway, negative regulation of BMK signalling pathway, negative regulation of BMK1 cascade, negative regulation of ERK5 signaling pathway, negative regulation of MAPK7 cascade, inhibition of BMK cascade Relationships: is a type of negative regulation of MAPK cascade [GO:0043409]; is a type of regulation of ERK5 cascade [GO:0070376]; negatively regulates ERK5 cascade [GO:0070375]